{
  "term_label": "aggrephagy",
  "term_id": "GO:0035973",
  "gene_name": "Cysteine protease ATG4D",
  "gene": "UniProtKB:Q86TL0",
  "gene_symbol": "ATG4D"
}